{
  "term_id": "GO:0006122",
  "term_label": "mitochondrial electron transport, ubiquinol to cytochrome c",
  "gene_name": "Cytochrome b",
  "gene": "UniProtKB:P00156",
  "gene_symbol": "MT-CYB"
}